{
  "gene_name": "Beta-defensin 134",
  "gene_symbol": "DEFB134",
  "gene": "UniProtKB:Q4QY38",
  "term_label": "Unknown molecular function",
  "term_id": "UNKNOWN:0001"
}